{
  "gene_name": "Troponin C, slow skeletal and cardiac muscles",
  "term_id": "GO:0060048",
  "gene": "UniProtKB:P63316",
  "gene_symbol": "TNNC1",
  "term_label": "cardiac muscle contraction"
}